stamen morphogenesis [GO:0048448] (biological process) Relationships: is a type of floral organ morphogenesis [GO:0048444]; is part of stamen development [GO:0048443] Sources: GOC:go_curators Definition: The process in which the anatomical structures of the stamen are generated and organized.